{
  "gene_name": "Calcium_calmodulin-dependent protein kinase type II subunit beta",
  "term_label": "regulation of protein localization to plasma membrane",
  "gene_symbol": "CAMK2B",
  "gene": "UniProtKB:Q13554",
  "term_id": "GO:1903076"
}